regulation of mesenchymal stem cell migration [GO:1905320] (biological process) Relationships: is a type of regulation of cell migration [GO:0030334]; regulates mesenchymal stem cell migration [GO:1905319] Subtypes: negative regulation of mesenchymal stem cell migration [GO:1905321], positive regulation of mesenchymal stem cell migration [GO:1905322] References: PMID:26846297 Sources: GOC:TermGenie, GO_REF:0000058 Definition: Any process that modulates the frequency, rate or extent of mesenchymal stem cell migration.